{
  "term_id": "UNKNOWN:0003",
  "gene": "UniProtKB:Q5T7P6",
  "term_label": "Unknown cellular component",
  "gene_symbol": "TMEM78",
  "gene_name": "Transmembrane protein 78"
}